{
  "gene_symbol": "POLD1",
  "term_label": "base-excision repair, gap-filling",
  "term_id": "GO:0006287",
  "gene": "UniProtKB:P28340",
  "gene_name": "DNA polymerase delta catalytic subunit"
}